{
  "term_label": "DNA-binding transcription factor activity, RNA polymerase II-specific",
  "gene_name": "Zinc finger protein 614",
  "gene": "UniProtKB:Q8N883",
  "term_id": "GO:0000981",
  "gene_symbol": "ZNF614"
}